{
  "term_id": "GO:0005938",
  "gene": "UniProtKB:P30622",
  "term_label": "cell cortex",
  "gene_name": "CAP-Gly domain-containing linker protein 1",
  "gene_symbol": "CLIP1"
}